{
  "gene_name": "Immunoglobulin heavy joining 5 (Fragment)",
  "term_id": "UNKNOWN:0001",
  "term_label": "Unknown molecular function",
  "gene": "UniProtKB:A0A0J9YVP9",
  "gene_symbol": "IGHJ5"
}